vanillin metabolic process [GO:0018982] (biological process) Definition: The chemical reactions and pathways involving vanillin, an aromatic hydrocarbon which occurs naturally in black vanilla bean pods and can be obtained as a by-product of the pulp and paper industry by the oxidative breakdown of lignin. Also known as: vanillic aldehyde metabolic process, vanillic aldehyde metabolism, vanillin metabolism Relationships: is a type of aldehyde metabolic process [GO:0006081]; is a type of GO:0018958; is_a GO:0042537 Sources: GOC:jl Subtypes: vanillin biosynthetic process [GO:0042189], vanillin catabolic process [GO:0042190]